viral genome replication [GO:0019079] (BP) Relationships: is a type of viral process [GO:0016032]; is part of viral life cycle [GO:0019058] Definition: Any process involved directly in viral genome replication, including viral nucleotide metabolism. Also known as: viral replication, sigma virus replication Sources: ISBN:0781702534 Regulation: negatively regulated by host-mediated suppression of viral genome replication [GO:0044828]; regulated by regulation of viral genome replication [GO:0045069]; positively regulated by positive regulation of viral genome replication [GO:0045070]; negatively regulated by negative regulation of viral genome replication [GO:0045071] Subtypes: viral DNA genome replication [GO:0039693], GO:0039694